{
  "term_label": "regulation of DNA-templated transcription",
  "gene_name": "Zinc finger protein 726",
  "term_id": "GO:0006355",
  "gene_symbol": "ZNF726",
  "gene": "UniProtKB:A6NNF4"
}